{
  "term_label": "digestive tract development",
  "term_id": "GO:0048565",
  "gene": "UniProtKB:O14627",
  "gene_name": "Homeobox protein CDX-4",
  "gene_symbol": "CDX4"
}